{
  "term_label": "heterochromatin formation",
  "gene": "UniProtKB:Q8TBE0",
  "gene_symbol": "BAHD1",
  "term_id": "GO:0031507",
  "gene_name": "Bromo adjacent homology domain-containing 1 protein"
}